selenocysteine methyltransferase activity [GO:0016205] (molecular function) Relationships: is a type of Se-methyltransferase activity [GO:0051995] Definition: Catalysis of the reaction: selenocysteine + S-adenosyl-L-methionine = Se-methylselenocysteine + S-adenosyl-homocysteine. References: PMID:10026151 Sources: EC:2.1.1.280